{
  "term_label": "calcium channel activity",
  "term_id": "GO:0005262",
  "gene_symbol": "GRINA",
  "gene_name": "Protein lifeguard 1",
  "gene": "UniProtKB:Q7Z429"
}